{
  "term_label": "plasma membrane",
  "gene_symbol": "PIP5K1B",
  "gene": "UniProtKB:O14986",
  "term_id": "GO:0005886",
  "gene_name": "Phosphatidylinositol 4-phosphate 5-kinase type-1 beta"
}